{
  "gene_name": "Putative coiled-coil domain-containing protein 144C",
  "gene_symbol": "CCDC144CP",
  "term_id": "UNKNOWN:0003",
  "gene": "UniProtKB:Q8IYA2",
  "term_label": "Unknown cellular component"
}